{
  "term_label": "Unknown cellular component",
  "gene_symbol": "TEX36",
  "gene_name": "Testis-expressed protein 36",
  "gene": "UniProtKB:Q5VZQ5",
  "term_id": "UNKNOWN:0003"
}